positive regulation of lipophagy [GO:1904504] (biological process) Definition: Any process that activates or increases the frequency, rate or extent of lipophagy. References: PMID:25383539 Sources: GOC:TermGenie, GOC:autophagy, GOC:dph, GO_REF:0000058 Also known as: up regulation of lipophagy, up-regulation of lipophagy, upregulation of lipophagy, activation of lipophagy Relationships: is a type of positive regulation of macroautophagy [GO:0016239]; is a type of regulation of lipophagy [GO:1904502]; RO_0002213 GO:0061724